response to lipoteichoic acid [GO:0070391] (BP) Also known as: response to LTA Definition: Any process that results in a change in state or activity of an organism (in terms of movement, secretion, enzyme production, gene expression, etc.) as a result of a lipoteichoic acid stimulus; lipoteichoic acid is a major component of the cell wall of gram-positive bacteria and typically consists of a chain of glycerol-phosphate repeating units linked to a glycolipid anchor. References: PMID:14665680, PMID:16020688 Sources: GOC:add Relationships: is a type of response to molecule of bacterial origin [GO:0002237]; is a type of response to oxygen-containing compound [GO:1901700] Subtypes: detection of lipoteichoic acid [GO:0070392], cellular response to lipoteichoic acid [GO:0071223]